{
  "gene_name": "Nuclear receptor subfamily 5 group A member 2",
  "gene_symbol": "NR5A2",
  "gene": "UniProtKB:O00482",
  "term_label": "RNA polymerase II transcription regulator complex",
  "term_id": "GO:0090575"
}